homotypic cell-cell adhesion [GO:0034109] (biological process) Regulation: regulated by regulation of homotypic cell-cell adhesion [GO:0034110]; negatively regulated by negative regulation of homotypic cell-cell adhesion [GO:0034111]; positively regulated by positive regulation of homotypic cell-cell adhesion [GO:0034112] Note: Note that this term is not synonymous with 'homophilic cell adhesion ; GO:0007156'; the process may occur by homophilic or heterophilic mechanisms. Sources: GOC:add Relationships: is a type of cell-cell adhesion [GO:0098609] Subtypes: cardioblast cell midline fusion [GO:0003317], GO:0034117, platelet aggregation [GO:0070527], cardiac muscle cell-cardiac muscle cell adhesion [GO:0086042], intermicrovillar adhesion [GO:0090675] Definition: The attachment of a cell to a second cell of the identical type via adhesion molecules.